{
  "term_id": "GO:0050428",
  "gene_symbol": "PAPSS2",
  "gene_name": "Bifunctional 3'-phosphoadenosine 5'-phosphosulfate synthase 2",
  "gene": "UniProtKB:O95340",
  "term_label": "3'-phosphoadenosine 5'-phosphosulfate biosynthetic process"
}